tRNA (adenine(58)-N1)-methyltransferase activity [GO:0160107] (molecular function) Definition: Catalysis of the reaction: adenosine(58) in tRNA + S-adenosyl-L-methionine = H+ + N(1)-methyladenosine(58) in tRNA + S-adenosyl-L-homocysteine. Relationships: is a type of tRNA (adenine) methyltransferase activity [GO:0016426] Sources: EC:2.1.1.220 Also known as: tRNA (adenine(58)-N(1))-methyltransferase activity, tRNA (m(1)A(58)) methyltransferase, tRNA m(1)A(58) methyltransferase